prostaglandin-A1 delta-isomerase activity [GO:0050219] (molecular function) Relationships: is a type of intramolecular oxidoreductase activity, transposing C=C bonds [GO:0016863] Definition: Catalysis of the reaction: prostaglandin A1 = prostaglandin C1. Also known as: prostaglandin-A1 D-isomerase activity, (13E)-(15S)-15-hydroxy-9-oxoprosta-10,13-dienoate delta10-delta11-isomerase activity, prostaglandin A isomerase activity Sources: RHEA:10460